myosin phosphatase activity [GO:0017018] (molecular function) Relationships: is a type of GO:0004722 Sources: EC:3.1.3.16 Definition: Catalysis of the reaction: phosphomyosin + H2O = myosin + phosphate. Also known as: myosin phosphatase, intrinsic catalyst activity, myosin phosphatase myosin binding Regulation: regulated by myosin phosphatase regulator activity [GO:0017020]